{
  "gene_name": "Hepatic and glial cell adhesion molecule",
  "term_label": "Unknown molecular function",
  "gene_symbol": "HEPACAM",
  "gene": "UniProtKB:Q14CZ8",
  "term_id": "UNKNOWN:0001"
}